{
  "gene_symbol": "GRM3",
  "gene": "UniProtKB:Q14832",
  "term_id": "GO:0005886",
  "term_label": "plasma membrane",
  "gene_name": "Metabotropic glutamate receptor 3"
}